{
  "term_id": "GO:0050853",
  "term_label": "B cell receptor signaling pathway",
  "gene_symbol": "BMX",
  "gene": "UniProtKB:P51813",
  "gene_name": "Cytoplasmic tyrosine-protein kinase BMX"
}